{
  "term_id": "GO:0006508",
  "gene": "UniProtKB:Q9UKF2",
  "gene_name": "Disintegrin and metalloproteinase domain-containing protein 30",
  "term_label": "proteolysis",
  "gene_symbol": "ADAM30"
}